{
  "gene_symbol": "HYI",
  "term_id": "GO:0008903",
  "gene_name": "Putative hydroxypyruvate isomerase",
  "term_label": "hydroxypyruvate isomerase activity",
  "gene": "UniProtKB:Q5T013"
}